{
  "term_id": "UNKNOWN:0001",
  "term_label": "Unknown molecular function",
  "gene_name": "Multiple PDZ domain protein",
  "gene": "UniProtKB:O75970",
  "gene_symbol": "MPDZ"
}